ulvan lyase activity [GO:0052763] (molecular function) References: PMID:9468631 Sources: GOC:mengo_curators Relationships: is_a GO:0016837 Definition: Catalysis of the cleavage of a carbon-oxygen bond in ulvan, a carbohydrate composed of a repeating structure of [->4)-beta-D-GlcA-(1,4)-alpha-L-Rha 3S-(1->4)-alpha-L-IdoA-(1->4)-alpha-L-Rha 3S-(1-]n. Continued digest of ulvan with an enzyme that can catalyze this reaction results in ulvanobiouronic acid A 3-sulfate [->4)-beta-D-GlcpA-(1->4)-alpha-L-Rhap 3-sulfate-(1-]n with 4-deoxy-L-threo-hex-4-enopyranosiduronic acid at the non-reducing end.